{
  "term_id": "GO:0005789",
  "term_label": "endoplasmic reticulum membrane",
  "gene_name": "Erlin-1",
  "gene": "UniProtKB:O75477",
  "gene_symbol": "ERLIN1"
}